{
  "gene_symbol": "VCAN",
  "term_label": "perineuronal net",
  "gene": "UniProtKB:P13611",
  "term_id": "GO:0072534",
  "gene_name": "Versican core protein"
}